negative regulation of protein ubiquitination [GO:0031397] (biological process) Definition: Any process that stops, prevents, or reduces the frequency, rate or extent of the addition of ubiquitin groups to a protein. Also known as: down regulation of protein ubiquitination, down-regulation of protein ubiquitination, downregulation of protein ubiquitination, inhibition of protein ubiquitination Sources: GOC:mah Relationships: is a type of regulation of protein ubiquitination [GO:0031396]; is a type of negative regulation of protein modification by small protein conjugation or removal [GO:1903321]; negatively regulates protein ubiquitination [GO:0016567] Subtypes: negative regulation of ubiquitin-protein transferase activity [GO:0051444], negative regulation of protein monoubiquitination [GO:1902526], negative regulation of protein polyubiquitination [GO:1902915], GO:1905524